{
  "term_label": "Unknown biological process",
  "gene_name": "LINE-1 retrotransposable element ORF2 protein",
  "term_id": "UNKNOWN:0002",
  "gene": "UniProtKB:O00370",
  "gene_symbol": "O00370"
}